{
  "gene_symbol": "IGHG1",
  "gene": "UniProtKB:P01857",
  "term_label": "immunoglobulin receptor binding",
  "term_id": "GO:0034987",
  "gene_name": "Immunoglobulin heavy constant gamma 1"
}